{
  "gene_name": "Probable ATP-dependent RNA helicase DDX28",
  "term_id": "GO:0005739",
  "gene_symbol": "DDX28",
  "term_label": "mitochondrion",
  "gene": "UniProtKB:Q9NUL7"
}